xyloglucan biosynthetic process [GO:0009969] (biological process) Relationships: is a type of glucan biosynthetic process [GO:0009250]; is a type of xyloglucan metabolic process [GO:0010411] Sources: GOC:sm Definition: The chemical reactions and pathways resulting in the formation of xyloglucan, the cross-linking glycan composed of (1->4)-beta-D glucan backbone substituted at regular intervals with beta-D-xylosyl-(1->6) residues, which is present in the primary cell wall of most higher plants. Also known as: xyloglucan anabolism, xyloglucan biosynthesis, xyloglucan formation, xyloglucan synthesis